{
  "gene_symbol": "PPP1CB",
  "gene": "UniProtKB:P62140",
  "gene_name": "Serine_threonine-protein phosphatase PP1-beta catalytic subunit",
  "term_label": "nucleus",
  "term_id": "GO:0005634"
}